positive regulation of ERBB3 signaling pathway [GO:1905580] (biological process) Relationships: is a type of GO:1901186; is a type of regulation of ERBB3 signaling pathway [GO:1905578]; positively regulates ERBB3 signaling pathway [GO:0038129] Also known as: positive regulation of ERBB3 signalling pathway, positive regulation of HER3 signaling pathway, positive regulation of receptor tyrosine-protein kinase erbB-3 signaling pathway, up regulation of ERBB3 signaling pathway, up regulation of ERBB3 signalling pathway, up regulation of HER3 signaling pathway, up regulation of receptor tyrosine-protein kinase erbB-3 signaling pathway, up-regulation of ERBB3 signaling pathway, up-regulation of ERBB3 signalling pathway, up-regulation of HER3 signaling pathway, up-regulation of receptor tyrosine-protein kinase erbB-3 signaling pathway, upregulation of ERBB3 signaling pathway, upregulation of ERBB3 signalling pathway, upregulation of HER3 signaling pathway, upregulation of receptor tyrosine-protein kinase erbB-3 signaling pathway, activation of ERBB3 signaling pathway, activation of ERBB3 signalling pathway, activation of HER3 signaling pathway, activation of receptor tyrosine-protein kinase erbB-3 signaling pathway References: PMID:27353365 Sources: GOC:TermGenie, GOC:als, GO_REF:0000058 Definition: Any process that activates or increases the frequency, rate or extent of ERBB3 signaling pathway.